{
  "gene_symbol": "WIPI1",
  "term_label": "protein-macromolecule adaptor activity",
  "gene": "UniProtKB:Q5MNZ9",
  "gene_name": "WD repeat domain phosphoinositide-interacting protein 1",
  "term_id": "GO:0030674"
}